nucleoside triphosphate adenylate kinase activity [GO:0046899] (MF) Also known as: nucleoside triphosphate-adenosine monophosphate transphosphorylase activity, nucleoside-triphosphate-adenylate kinase activity, GTP:AMP phosphotransferase, guanosine triphosphate-adenylate kinase, isozyme 3 of adenylate kinase activity, nucleoside-triphosphate:AMP phosphotransferase activity Sources: EC:2.7.4.10 Relationships: is_a phosphotransferase activity, phosphate group as acceptor [GO:0016776]; is a type of GO:0019205 Definition: Catalysis of the reaction: nucleoside triphosphate + AMP = nucleoside diphosphate + ADP.